23S rRNA (adenosine(1067)-2'-O)-methyltransferase activity [GO:0030743] (molecular function) Definition: Catalysis of the reaction: adenosine(1067) in 23S rRNA + S-adenosyl-L-methionine = 2'-O-methyladenosine(1067) in 23S rRNA + H+ + S-adenosyl-L-homocysteine. Sources: EC:2.1.1.230 Also known as: thiostrepton-resistance methylase activity, RNA-pentose methylase activity, S-adenosyl-L-methionine:rRNA (adenosine-2'-O)-methyltransferase activity, rRNA adenosine 2'-methylase activity, ribosomal ribonucleate adenosine 2'-methyltransferase activity Relationships: is a type of rRNA (adenine) methyltransferase activity [GO:0016433]; is a type of RNA 2'-O-methyltransferase activity [GO:0062105]